polarity specification of adaxial/abaxial axis [GO:0009944] (biological process) Definition: The process resulting in the establishment of polarity along the adaxial/abaxial axis. Adaxial refers to being situated toward an axis of an anatomical structure. Abaxial refers to being situated away from an axis of an anatomical structure. Sources: GOC:dph, GOC:tb Relationships: is a type of specification of axis polarity [GO:0065001]; is part of adaxial/abaxial axis specification [GO:0009943]